{
  "gene": "UniProtKB:Q9H7B7",
  "gene_symbol": "PKD1L1-AS1",
  "term_label": "Unknown molecular function",
  "term_id": "UNKNOWN:0001",
  "gene_name": "Putative uncharacterized protein PKD1L1-AS1"
}